polygalacturonase activity [GO:0004650] (molecular function) Sources: EC:3.2.1.15 Relationships: is a type of hydrolase activity, hydrolyzing O-glycosyl compounds [GO:0004553] Definition: Catalysis of the random hydrolysis of (1->4)-alpha-D-galactosiduronic linkages in pectate and other galacturonans. Regulation: negatively regulated by GO:0090353 Also known as: endo-D-galacturonase activity, endo-polygalacturonase activity, endogalacturonase activity, endopolygalacturonase activity, poly(1,4-alpha-D-galacturonide) glycanohydrolase activity, poly-alpha-1,4-galacturonide glycanohydrolase activity, pectin depolymerase activity, pectinase activity, pectin hydrolase activity, pectin polygalacturonase activity, pectolase activity